{
  "gene": "UniProtKB:Q8ND07",
  "term_id": "UNKNOWN:0001",
  "gene_symbol": "BBOF1",
  "gene_name": "Basal body-orientation factor 1",
  "term_label": "Unknown molecular function"
}